{
  "gene": "UniProtKB:Q9NYK5",
  "term_id": "UNKNOWN:0001",
  "gene_symbol": "MRPL39",
  "gene_name": "Large ribosomal subunit protein mL39",
  "term_label": "Unknown molecular function"
}